{
  "gene": "UniProtKB:P63145",
  "term_id": "UNKNOWN:0003",
  "term_label": "Unknown cellular component",
  "gene_symbol": "ERVK-24",
  "gene_name": "Endogenous retrovirus group K member 24 Gag polyprotein"
}